{
  "gene": "UniProtKB:P21266",
  "gene_name": "Glutathione S-transferase Mu 3",
  "gene_symbol": "GSTM3",
  "term_id": "GO:0006749",
  "term_label": "glutathione metabolic process"
}